{
  "gene_symbol": "VMP1",
  "term_label": "Unknown molecular function",
  "gene": "UniProtKB:Q96GC9",
  "gene_name": "Vacuole membrane protein 1",
  "term_id": "UNKNOWN:0001"
}